{
  "term_label": "oxygen carrier activity",
  "gene_symbol": "HBG1",
  "term_id": "GO:0005344",
  "gene_name": "Hemoglobin subunit gamma-1",
  "gene": "UniProtKB:P69891"
}